{
  "term_id": "GO:0030667",
  "term_label": "secretory granule membrane",
  "gene": "UniProtKB:Q6UVY6",
  "gene_name": "DBH-like monooxygenase protein 1",
  "gene_symbol": "MOXD1"
}